{
  "gene": "UniProtKB:Q02846",
  "gene_name": "Retinal guanylyl cyclase 1",
  "term_id": "GO:0001653",
  "term_label": "peptide receptor activity",
  "gene_symbol": "GUCY2D"
}